{
  "term_label": "plasma membrane",
  "term_id": "GO:0005886",
  "gene_name": "Membrane-spanning 4-domains subfamily A member 10",
  "gene": "UniProtKB:Q96PG2",
  "gene_symbol": "MS4A10"
}